{
  "gene_name": "Protein PRRC2B",
  "gene": "UniProtKB:Q5JSZ5",
  "term_id": "UNKNOWN:0001",
  "gene_symbol": "PRRC2B",
  "term_label": "Unknown molecular function"
}